{
  "term_id": "GO:0006888",
  "gene_symbol": "TMED2",
  "gene_name": "Transmembrane emp24 domain-containing protein 2",
  "gene": "UniProtKB:Q15363",
  "term_label": "endoplasmic reticulum to Golgi vesicle-mediated transport"
}